alpha-farnesene synthase activity [GO:0052578] (molecular function) Sources: MetaCyc:RXN-8574 Also known as: (E,E)-alpha-farnesene synthase activity Definition: Catalysis of the reaction: 2-trans,6-trans-farnesyl diphosphate = (E,E)-alpha-farnesene + diphosphate. Relationships: is a type of GO:0010334